{
  "term_label": "Unknown molecular function",
  "gene_symbol": "CEP20",
  "term_id": "UNKNOWN:0001",
  "gene": "UniProtKB:Q96NB1",
  "gene_name": "Centrosomal protein 20"
}